{
  "term_id": "GO:0048705",
  "gene_name": "Collagen alpha-1(XI) chain",
  "gene": "UniProtKB:P12107",
  "term_label": "skeletal system morphogenesis",
  "gene_symbol": "COL11A1"
}